{
  "term_id": "UNKNOWN:0001",
  "gene": "UniProtKB:O96015",
  "term_label": "Unknown molecular function",
  "gene_symbol": "DNAL4",
  "gene_name": "Dynein axonemal light chain 4"
}